{
  "gene": "UniProtKB:O76076",
  "gene_symbol": "CCN5",
  "term_label": "signal transduction",
  "term_id": "GO:0007165",
  "gene_name": "CCN family member 5"
}